negative regulation of filamentous growth of a population of unicellular organisms in response to chemical stimulus [GO:1900438] (biological process) Definition: Any process that stops, prevents or reduces the frequency, rate or extent of filamentous growth of a population of unicellular organisms in response to chemical stimulus. Sources: GOC:TermGenie, GOC:di Also known as: down regulation of filamentous growth of a population of unicellular organisms in response to chemical stimulus, down-regulation of filamentous growth of a population of unicellular organisms in response to chemical stimulus, downregulation of filamentous growth of a population of unicellular organisms in response to chemical stimulus, inhibition of filamentous growth of a population of unicellular organisms in response to chemical stimulus Relationships: is a type of negative regulation of response to stimulus [GO:0048585]; is a type of negative regulation of filamentous growth of a population of unicellular organisms [GO:1900429]; is a type of regulation of filamentous growth of a population of unicellular organisms in response to chemical stimulus [GO:1900437]; negatively regulates filamentous growth of a population of unicellular organisms in response to chemical stimulus [GO:0036171]